{
  "term_label": "Unknown cellular component",
  "gene": "UniProtKB:Q5EB52",
  "term_id": "UNKNOWN:0003",
  "gene_symbol": "MEST",
  "gene_name": "Mesoderm-specific transcript homolog protein"
}